columnar/cuboidal epithelial cell maturation [GO:0002069] (biological process) Subtypes: GO:0002071, intestinal epithelial cell maturation [GO:0060574] Definition: The developmental process, independent of morphogenetic (shape) change, that is required for a columna/cuboidal epithelial cell to attain its fully functional state. A columnar/cuboidal epithelial cell is a cell usually found in a two dimensional sheet with a free surface. Columnar/cuboidal epithelial cells take on the shape of a column or cube. Sources: GOC:dph Relationships: is a type of epithelial cell maturation [GO:0002070]; is part of columnar/cuboidal epithelial cell development [GO:0002066]